{
  "gene_symbol": "MOGAT1",
  "term_label": "diacylglycerol O-acyltransferase activity",
  "gene": "UniProtKB:Q96PD6",
  "gene_name": "2-acylglycerol O-acyltransferase 1",
  "term_id": "GO:0004144"
}